{
  "term_label": "synapse",
  "gene_symbol": "KIDINS220",
  "term_id": "GO:0045202",
  "gene_name": "Kinase D-interacting substrate of 220 kDa",
  "gene": "UniProtKB:Q9ULH0"
}